symbiont-mediated evasion of host restriction-modification system [GO:0099018] (biological process) Also known as: evasion of host restriction-modification system, restriction-modification system evasion by virus, evasion by virus of host restriction-modification system Relationships: is a type of symbiont-mediated evasion of recognition by host innate immune effector [GO:0141177] References: PMID:20348932, PMID:23979432, PMID:24123737 Sources: VZ:3966 Definition: A process by which a symbiont evades the DNA restriction modification system of its host. This process occurs in phages to protein themselves from bacterial restriction enzyme systems. Some viruses encode their own methyltransferase in order to protect their genome from host restriction enzymes. Others directly inhibit restriction enzymes while some use unusual bases in their genome to avoid restriction.